{
  "gene_name": "Gamma-aminobutyric acid receptor subunit gamma-3",
  "term_id": "GO:1904862",
  "gene": "UniProtKB:Q99928",
  "term_label": "inhibitory synapse assembly",
  "gene_symbol": "GABRG3"
}